{
  "gene": "UniProtKB:Q9Y5K2",
  "term_id": "GO:0005615",
  "gene_name": "Kallikrein-4",
  "term_label": "extracellular space",
  "gene_symbol": "KLK4"
}